{
  "term_id": "GO:0006682",
  "term_label": "galactosylceramide biosynthetic process",
  "gene_symbol": "B4GALT3",
  "gene": "UniProtKB:O60512",
  "gene_name": "Beta-1,4-galactosyltransferase 3"
}